{
  "gene_name": "T-complex protein 10A homolog 1",
  "term_label": "Unknown biological process",
  "gene_symbol": "TCP10L",
  "term_id": "UNKNOWN:0002",
  "gene": "UniProtKB:Q8TDR4"
}